{
  "term_id": "GO:0007169",
  "gene_symbol": "SAMD12",
  "gene_name": "Sterile alpha motif domain-containing protein 12",
  "gene": "UniProtKB:Q8N8I0",
  "term_label": "cell surface receptor protein tyrosine kinase signaling pathway"
}